{
  "term_id": "GO:1904315",
  "gene_name": "Glutamate receptor ionotropic, delta-1",
  "term_label": "transmitter-gated monoatomic ion channel activity involved in regulation of postsynaptic membrane potential",
  "gene": "UniProtKB:Q9ULK0",
  "gene_symbol": "GRID1"
}